{
  "gene_name": "Endoplasmic reticulum lectin 1",
  "term_id": "GO:0030970",
  "gene_symbol": "ERLEC1",
  "gene": "UniProtKB:Q96DZ1",
  "term_label": "retrograde protein transport, ER to cytosol"
}